{
  "gene_name": "Leucine-rich repeat-containing protein 7",
  "term_label": "adherens junction",
  "gene": "UniProtKB:Q96NW7",
  "term_id": "GO:0005912",
  "gene_symbol": "LRRC7"
}